{
  "gene_name": "NF-kappa-B inhibitor-interacting Ras-like protein 2",
  "term_id": "GO:0032794",
  "term_label": "GTPase activating protein binding",
  "gene_symbol": "NKIRAS2",
  "gene": "UniProtKB:Q9NYR9"
}